{
  "gene_name": "14-3-3 protein sigma",
  "term_label": "intracellular protein localization",
  "gene": "UniProtKB:P31947",
  "term_id": "GO:0008104",
  "gene_symbol": "SFN"
}